regulation of hypoxia-induced intrinsic apoptotic signaling pathway [GO:1903297] (biological process) Relationships: is a type of regulation of intrinsic apoptotic signaling pathway [GO:2001242]; regulates intrinsic apoptotic signaling pathway in response to hypoxia [GO:1990144] Also known as: regulation of hypoxic stress-induced intrinsic apoptotic signaling pathway, regulation of intrinsic apoptotic signaling pathway in response to hypoxia, regulation of hypoxia-induced apoptosis Subtypes: negative regulation of hypoxia-induced intrinsic apoptotic signaling pathway [GO:1903298] Definition: Any process that modulates the frequency, rate or extent of hypoxia-induced intrinsic apoptotic signaling pathway. Sources: GOC:PARL, GOC:TermGenie, GOC:bf, GO_REF:0000058